{
  "gene_name": "Protein SCAI",
  "gene_symbol": "SCAI",
  "term_label": "Unknown biological process",
  "term_id": "UNKNOWN:0002",
  "gene": "UniProtKB:Q8N9R8"
}